{
  "term_id": "GO:0060337",
  "gene_symbol": "IFNA17",
  "gene_name": "Interferon alpha-17",
  "term_label": "type I interferon-mediated signaling pathway",
  "gene": "UniProtKB:P01571"
}